chloride:proton antiporter activity [GO:0062158] (MF) References: PMID:14985752 Definition: Enables the transfer of a solute or solutes from one side of a membrane to the other according to the reaction: chloride(out) + proton(in) = chloride(in) + proton(out). Relationships: is a type of solute:inorganic anion antiporter activity [GO:0005452]; is a type of proton transmembrane transporter activity [GO:0015078]; is_a chloride transmembrane transporter activity [GO:0015108]